{
  "term_id": "GO:0005886",
  "gene_name": "Alpha-1B adrenergic receptor",
  "gene": "UniProtKB:P35368",
  "gene_symbol": "ADRA1B",
  "term_label": "plasma membrane"
}